{
  "term_label": "snRNA 3'-end processing",
  "gene_name": "Integrator complex subunit 5",
  "gene": "UniProtKB:Q6P9B9",
  "gene_symbol": "INTS5",
  "term_id": "GO:0034472"
}